{
  "term_id": "UNKNOWN:0002",
  "gene_symbol": "EFCAB10",
  "term_label": "Unknown biological process",
  "gene_name": "EF-hand calcium-binding domain-containing protein 10",
  "gene": "UniProtKB:A6NFE3"
}